{
  "term_id": "GO:0006357",
  "gene_symbol": "RLF",
  "term_label": "regulation of transcription by RNA polymerase II",
  "gene": "UniProtKB:Q13129",
  "gene_name": "Zinc finger protein Rlf"
}